putrescine carbamoyltransferase activity [GO:0050231] (molecular function) Also known as: PTCase activity, carbamoyl-phosphate:putrescine carbamoyltransferase activity, putrescine synthase activity, putrescine transcarbamylase activity Relationships: is a type of carboxyl- or carbamoyltransferase activity [GO:0016743] Definition: Catalysis of the reaction: carbamoyl phosphate + putrescine = N-carbamoylputrescine + H+ + phosphate. Sources: EC:2.1.3.6, RHEA:21936